{
  "gene_symbol": "SCN3A",
  "gene": "UniProtKB:Q9NY46",
  "term_label": "voltage-gated sodium channel activity",
  "term_id": "GO:0005248",
  "gene_name": "Sodium channel protein type 3 subunit alpha"
}